interstitial matrix [GO:0005614] (cellular component) References: PMID:33605520, PMID:39223427, PMID:8450001 Definition: A type of extracellular matrix found in interstitial connective tissue, characterized by the presence of fibronectins, proteoglycans, and types I, III, V, VI, VII and XII collagens. Relationships: is a type of extracellular matrix [GO:0031012]